{
  "term_id": "GO:0030382",
  "gene_name": "Spermatogenesis-associated protein 19, mitochondrial",
  "gene_symbol": "SPATA19",
  "gene": "UniProtKB:Q7Z5L4",
  "term_label": "sperm mitochondrion organization"
}